{
  "gene": "UniProtKB:O76039",
  "term_label": "nucleus",
  "term_id": "GO:0005634",
  "gene_name": "Cyclin-dependent kinase-like 5",
  "gene_symbol": "CDKL5"
}